dCTP biosynthetic process [GO:0006242] (biological process) Relationships: is a type of GO:0009212; is a type of GO:0009221; is a type of dCTP metabolic process [GO:0046065] Also known as: dCTP anabolism, dCTP biosynthesis, dCTP formation, dCTP synthesis Sources: ISBN:0198506732 Definition: The chemical reactions and pathways resulting in the formation of dCTP, deoxycytidine triphosphate.